chromosome segregation [GO:0007059] (biological process) Also known as: chromosome division, chromosome transmission Relationships: is a type of cell cycle process [GO:0022402] Sources: GOC:jl, GOC:mah, GOC:mtg_cell_cycle, GOC:vw Subtypes: nuclear chromosome segregation [GO:0098813] Regulation: regulated by GO:0051983; positively regulated by positive regulation of chromosome segregation [GO:0051984]; negatively regulated by negative regulation of chromosome segregation [GO:0051985] Definition: The process in which genetic material, in the form of chromosomes, is organized into specific structures and then physically separated and apportioned to two or more sets. In eukaryotes, chromosome segregation begins with the condensation of chromosomes, includes chromosome separation, and ends when chromosomes have completed movement to the spindle poles.